pre-mRNA 5'-splice site binding [GO:0030627] (molecular function) Also known as: pre-mRNA 5' splice site binding Definition: Binding to a pre-mRNA 5' splice site sequence. Sources: GOC:jl Relationships: is a type of pre-mRNA binding [GO:0036002]